{
  "gene_name": "Homeobox protein DLX-6",
  "term_id": "GO:0000981",
  "term_label": "DNA-binding transcription factor activity, RNA polymerase II-specific",
  "gene": "UniProtKB:P56179",
  "gene_symbol": "DLX6"
}